{
  "term_label": "axon",
  "gene": "UniProtKB:Q9UQ52",
  "gene_symbol": "CNTN6",
  "term_id": "GO:0030424",
  "gene_name": "Contactin-6"
}